{
  "term_label": "regulation of transcription by RNA polymerase II",
  "gene": "UniProtKB:B7ZLF3",
  "term_id": "GO:0006357",
  "gene_symbol": "LOC728743",
  "gene_name": "C2H2-type domain-containing protein"
}